{
  "gene": "UniProtKB:Q96BQ5",
  "gene_symbol": "CCDC127",
  "gene_name": "Coiled-coil domain-containing protein 127",
  "term_label": "Unknown cellular component",
  "term_id": "UNKNOWN:0003"
}